{
  "gene_symbol": "FBLL1",
  "term_id": "GO:0031167",
  "term_label": "rRNA methylation",
  "gene_name": "rRNA_tRNA 2'-O-methyltransferase fibrillarin-like protein 1",
  "gene": "UniProtKB:A6NHQ2"
}